{
  "gene_symbol": "SPN",
  "gene": "UniProtKB:P16150",
  "gene_name": "Leukosialin",
  "term_id": "GO:0007166",
  "term_label": "cell surface receptor signaling pathway"
}